positive regulation of gamma-aminobutyric acid uptake involved in transmission of nerve impulse [GO:0051950] (biological process) Definition: Any process that activates, maintains or increases the frequency, rate or extent of the directed movement of gamma-aminobutyric acid (GABA, 4-aminobutyrate) into a neuron or glial cell. Also known as: positive regulation of 4-aminobutyrate reuptake, positive regulation of 4-aminobutyrate uptake during transmission of nerve impulse, positive regulation of GABA reuptake, positive regulation of GABA uptake during transmission of nerve impulse, positive regulation of gamma-aminobutyric acid reuptake, positive regulation of gamma-aminobutyric acid uptake involved in conduction of nerve impulse, up regulation of gamma-aminobutyric acid uptake during transmission of nerve impulse, up-regulation of gamma-aminobutyric acid uptake during transmission of nerve impulse, upregulation of gamma-aminobutyric acid uptake during transmission of nerve impulse, activation of gamma-aminobutyric acid uptake during transmission of nerve impulse, stimulation of gamma-aminobutyric acid uptake during transmission of nerve impulse, positive regulation of gamma-aminobutyric acid uptake during transmission of nerve impulse Relationships: is a type of positive regulation of organic acid transport [GO:0032892]; is a type of positive regulation of amino acid uptake involved in synaptic transmission [GO:0051943]; is a type of GO:0051947; positively regulates gamma-aminobutyric acid reuptake [GO:0051936] Sources: GOC:ai